{
  "gene_name": "Olfactory receptor 1M1",
  "gene_symbol": "OR1M1",
  "term_label": "signal transduction",
  "term_id": "GO:0007165",
  "gene": "UniProtKB:Q8NGA1"
}